{
  "term_label": "replication fork processing",
  "gene_symbol": "FAM111A",
  "term_id": "GO:0031297",
  "gene_name": "Serine protease FAM111A",
  "gene": "UniProtKB:Q96PZ2"
}